{
  "gene_name": "Sodium_hydrogen exchanger 1",
  "term_label": "regulation of intracellular pH",
  "term_id": "GO:0051453",
  "gene_symbol": "SLC9A1",
  "gene": "UniProtKB:P19634"
}